negative regulation of amyloid-beta clearance [GO:1900222] (biological process) Sources: GOC:BHF, GOC:TermGenie Relationships: is a type of GO:0051241; is a type of regulation of amyloid-beta clearance [GO:1900221]; negatively regulates GO:0097242 Also known as: down regulation of beta-amyloid clearance, down-regulation of beta-amyloid clearance, downregulation of beta-amyloid clearance, negative regulation of beta-amyloid clearance, inhibition of beta-amyloid clearance Definition: Any process that stops, prevents or reduces the frequency, rate or extent of amyloid-beta clearance.